growth hormone receptor signaling pathway via JAK-STAT [GO:0060397] (biological process) Also known as: JAK-STAT cascade involved in growth hormone signalling pathway Relationships: is a type of growth hormone receptor signaling pathway [GO:0060396] Definition: The process in which STAT proteins (Signal Transducers and Activators of Transcription) are activated by members of the JAK (janus activated kinase) family of tyrosine kinases, following the binding of physiological ligands to the growth hormone receptor. Once activated, STATs dimerize and translocate to the nucleus and modulate the expression of target genes. References: PMID:11445442 Sources: GOC:BHF, GOC:dph